{
  "gene": "UniProtKB:P14174",
  "term_label": "phenylpyruvate tautomerase activity",
  "gene_name": "Macrophage migration inhibitory factor",
  "gene_symbol": "MIF",
  "term_id": "GO:0050178"
}